{
  "gene_name": "Zinc transporter ZIP6",
  "gene_symbol": "SLC39A6",
  "gene": "UniProtKB:Q13433",
  "term_label": "plasma membrane",
  "term_id": "GO:0005886"
}